{
  "gene": "UniProtKB:Q9HB65",
  "gene_name": "RNA polymerase II elongation factor ELL3",
  "gene_symbol": "ELL3",
  "term_id": "GO:0032968",
  "term_label": "positive regulation of transcription elongation by RNA polymerase II"
}